galactose transmembrane transporter activity [GO:0005354] (molecular function) Subtypes: GO:0015371, galactose:proton symporter activity [GO:0015517], galactose uniporter activity [GO:0050782], ABC-type D-galactofuranose transporter [GO:0103116] Sources: GOC:ai, GOC:mtg_transport, ISBN:0815340729 Definition: Enables the transfer of galactose from one side of a membrane to the other. D-galactose is widely distributed in combined form in plants, animals and microorganisms as a constituent of oligo- and polysaccharides; it also occurs in galactolipids and as its glucoside in lactose and melibiose. Relationships: is a type of hexose transmembrane transporter activity [GO:0015149]; is part of galactose transmembrane transport [GO:0015757] Also known as: galactose/glucose (methylgalactoside) porter activity